{
  "gene_symbol": "DYNC2I1",
  "term_id": "GO:0097546",
  "gene_name": "Cytoplasmic dynein 2 intermediate chain 1",
  "gene": "UniProtKB:Q8WVS4",
  "term_label": "ciliary base"
}